{
  "term_label": "cytoplasm",
  "gene": "UniProtKB:Q9ULI2",
  "term_id": "GO:0005737",
  "gene_symbol": "RIMKLB",
  "gene_name": "Beta-citrylglutamate synthase B"
}